{
  "gene_symbol": "ELOA2",
  "term_label": "Unknown molecular function",
  "term_id": "UNKNOWN:0001",
  "gene_name": "Elongin-A2",
  "gene": "UniProtKB:Q8IYF1"
}